{
  "gene": "UniProtKB:Q9P2R3",
  "term_id": "GO:0031267",
  "gene_name": "Rabankyrin-5",
  "term_label": "small GTPase binding",
  "gene_symbol": "ANKFY1"
}